{
  "term_label": "Rab-protein geranylgeranyltransferase complex",
  "gene_symbol": "RABGGTB",
  "gene": "UniProtKB:P53611",
  "term_id": "GO:0005968",
  "gene_name": "Geranylgeranyl transferase type-2 subunit beta"
}